{
  "gene_name": "COUP transcription factor 2",
  "term_label": "retinoic acid binding",
  "gene": "UniProtKB:P24468",
  "term_id": "GO:0001972",
  "gene_symbol": "NR2F2"
}